cellulose synthase complex [GO:0010330] (cellular component) Relationships: is a type of transferase complex [GO:1990234] References: PMID:12514238, PMID:18485800, PMID:21307367 Subtypes: primary cell wall cellulose synthase complex [GO:0044567], secondary cell wall cellulose synthase complex [GO:0044568] Also known as: CESA complex Definition: A large, multimeric protein complex, organized in a rosette, which catalyzes the biosynthesis of cellulose for the plant cell wall.